{
  "term_label": "metalloendopeptidase activity",
  "gene": "UniProtKB:Q9UKQ2",
  "term_id": "GO:0004222",
  "gene_symbol": "ADAM28",
  "gene_name": "Disintegrin and metalloproteinase domain-containing protein 28"
}